thiazole synthase activity [GO:1990107] (molecular function) Also known as: 1-deoxy-D-xylulose 5-phosphate:thiol sulfurtransferase activity Relationships: is a type of GO:0016783; is part of thiamine biosynthetic process [GO:0009228] Definition: Catalysis of the reaction: 1-deoxy-D-xylulose 5-phosphate + 2-iminoacetate + [sulfur-carrier protein ThiS]-C-terminal Gly-NH-CH2-C(O)SH = 2-[(2R,5Z)-2-carboxy-4-methylthiazol-5(2H)-ylidene]ethyl phosphate + [sulfur-carrier protein ThiS]-C-terminal Gly-Gly + 2 H+ + 2 H2O. Note: Part of the pathway for thiamine biosynthesis. References: PMID:22031445 Sources: RHEA:26297